6-endo-hydroxycineole dehydrogenase activity [GO:0045481] (molecular function) Relationships: is a type of oxidoreductase activity, acting on the CH-OH group of donors, NAD or NADP as acceptor [GO:0016616] Definition: Catalysis of the reaction: 6-endo-hydroxycineole + NAD+ = 6-oxocineole + H+ + NADH. Also known as: 6-endo-hydroxycineole:NAD+ 6-oxidoreductase activity Sources: EC:1.1.1.241, RHEA:11736